{
  "term_id": "GO:0046620",
  "gene": "UniProtKB:O95835",
  "gene_symbol": "LATS1",
  "term_label": "regulation of organ growth",
  "gene_name": "Serine_threonine-protein kinase LATS1"
}